regulation of chitin biosynthetic process [GO:0032883] (biological process) Definition: Any process that modulates the frequency, rate or extent of the chemical reactions and pathways resulting in the formation of chitin. Relationships: is a type of regulation of chitin metabolic process [GO:0032882]; is a type of regulation of polysaccharide biosynthetic process [GO:0032885]; regulates chitin biosynthetic process [GO:0006031] Also known as: regulation of chitin anabolism, regulation of chitin formation, regulation of chitin synthesis, regulation of chitin biosynthesis Sources: GOC:mah